{
  "term_id": "GO:0005886",
  "gene_symbol": "LRRN1",
  "gene": "UniProtKB:Q6UXK5",
  "term_label": "plasma membrane",
  "gene_name": "Leucine-rich repeat neuronal protein 1"
}